glycero-3-phosphocholine acyltransferase activity [GO:0106158] (molecular function) References: PMID:18430972, PMID:27758859 Sources: RHEA:58476 Definition: Catalysis of the reaction:acyl-CoA + glycerophosphocholine = CoA + 1-acyl-sn-glycero-3-phosphocholine. Relationships: is a type of GO:0016747 Also known as: GPACT activity, glycerophosphocholine O-acyltransferase activity